{
  "term_id": "GO:0042776",
  "gene_name": "ATP synthase subunit epsilon, mitochondrial",
  "gene_symbol": "ATP5F1E",
  "gene": "UniProtKB:P56381",
  "term_label": "proton motive force-driven mitochondrial ATP synthesis"
}